{
  "term_id": "GO:0014842",
  "gene": "UniProtKB:Q03181",
  "gene_symbol": "PPARD",
  "gene_name": "Peroxisome proliferator-activated receptor delta",
  "term_label": "regulation of skeletal muscle satellite cell proliferation"
}